bone trabecula formation [GO:0060346] (biological process) Definition: The process of creating a trabecula in the bone. A trabecula is a tissue element in the form of a small beam, strut or rod. Regulation: regulated by regulation of bone trabecula formation [GO:1900154]; negatively regulated by GO:1900155; positively regulated by GO:1900156 Also known as: bone trabeculation, skeletal trabecula formation, skeletal trabeculation, bone trabecula biogenesis, skeletal trabecula biogenesis Sources: GOC:dph Relationships: is a type of trabecula formation [GO:0060343]; is part of skeletal system morphogenesis [GO:0048705]; is part of bone trabecula morphogenesis [GO:0061430]